{
  "term_label": "heterotrimeric G-protein complex",
  "gene": "UniProtKB:P29992",
  "term_id": "GO:0005834",
  "gene_name": "Guanine nucleotide-binding protein subunit alpha-11",
  "gene_symbol": "GNA11"
}